{
  "gene": "UniProtKB:O75506",
  "gene_symbol": "HSBP1",
  "term_id": "GO:0005634",
  "gene_name": "Heat shock factor-binding protein 1",
  "term_label": "nucleus"
}